protein co-translational transfer of dolichol-linked oligosaccharide [GO:0180058] (biological process) Also known as: protein N-linked glycosylation via asparagine, co-translational, protein N-linked glycosylation via asparagine, cotranslational, protein cotranslational transfer of dolichol-linked oligosaccharide Definition: A N-linked protein glycosylation process in which the preassembled dolichol-linked oligosaccharide precursor is transfered post-translationally to an asparagine residue within the motif Asn-X-Ser/Thr of the target protein. This is mediated by the OSTA complex. References: PMID:19167329 Relationships: is a type of GO:0009101; is part of protein N-linked glycosylation [GO:0006487]